{
  "gene_symbol": "RANGAP1",
  "gene_name": "Ran GTPase-activating protein 1",
  "term_id": "GO:0005634",
  "gene": "UniProtKB:P46060",
  "term_label": "nucleus"
}